{
  "gene_name": "Remodeling and spacing factor 1",
  "gene": "UniProtKB:Q96T23",
  "term_label": "heterochromatin formation",
  "term_id": "GO:0031507",
  "gene_symbol": "RSF1"
}